{
  "term_label": "Unknown biological process",
  "gene_name": "HOXB-AS3 peptide",
  "gene_symbol": "HOXB-AS3",
  "gene": "UniProtKB:C0HLZ6",
  "term_id": "UNKNOWN:0002"
}